{
  "term_label": "endosomal transport",
  "gene": "UniProtKB:Q2VPB7",
  "gene_name": "AP-5 complex subunit beta-1",
  "gene_symbol": "AP5B1",
  "term_id": "GO:0016197"
}